{
  "gene_symbol": "UQCR10",
  "term_label": "Unknown molecular function",
  "term_id": "UNKNOWN:0001",
  "gene_name": "Cytochrome b-c1 complex subunit 9",
  "gene": "UniProtKB:Q9UDW1"
}